{
  "gene_symbol": "NLRP7",
  "term_id": "GO:0050727",
  "gene_name": "NACHT, LRR and PYD domains-containing protein 7",
  "term_label": "regulation of inflammatory response",
  "gene": "UniProtKB:Q8WX94"
}